{
  "term_id": "GO:0005886",
  "gene_name": "Stromal interaction molecule 2",
  "gene_symbol": "STIM2",
  "gene": "UniProtKB:Q9P246",
  "term_label": "plasma membrane"
}